{
  "gene_name": "Testis-expressed protein 51",
  "gene": "UniProtKB:A0A1B0GUA7",
  "term_id": "UNKNOWN:0001",
  "term_label": "Unknown molecular function",
  "gene_symbol": "TEX51"
}